positive regulation of germinal center formation [GO:0002636] (BP) Relationships: is a type of regulation of germinal center formation [GO:0002634]; is a type of positive regulation of adaptive immune response based on somatic recombination of immune receptors built from immunoglobulin superfamily domains [GO:0002824]; is a type of positive regulation of developmental process [GO:0051094]; positively regulates GO:0002467 Also known as: up regulation of germinal center formation, up-regulation of germinal center formation, upregulation of germinal center formation, activation of germinal center formation, stimulation of germinal center formation Sources: GOC:add Definition: Any process that activates or increases the frequency, rate, or extent of germinal center formation.